establishment of endothelial blood-brain barrier [GO:0014045] (biological process) Definition: Establishment of the endothelial barrier between the blood and the brain. The endothelial cells in the brain capillaries are packed tightly together preventing the passage of most molecules from the blood into the brain. Only lipid soluble molecules or those that are actively transported can pass through the blood-brain barrier. References: PMID:20080302, PMID:30280653 Sources: GOC:aruk, GOC:dgh, GOC:dph, GOC:sart Also known as: establishment of endothelial BBB, establishment of endothelial blood/brain barrier Relationships: is a type of establishment of blood-brain barrier [GO:0060856]; is a type of GO:0061028